{
  "gene_symbol": "OPN1MW",
  "term_id": "GO:0005886",
  "gene_name": "Medium-wave-sensitive opsin 1",
  "term_label": "plasma membrane",
  "gene": "UniProtKB:P04001"
}